{
  "gene_name": "Formin-binding protein 4",
  "gene_symbol": "FNBP4",
  "gene": "UniProtKB:Q8N3X1",
  "term_label": "Unknown biological process",
  "term_id": "UNKNOWN:0002"
}